{
  "gene": "UniProtKB:Q02156",
  "term_id": "GO:0004674",
  "gene_name": "Protein kinase C epsilon type",
  "term_label": "protein serine/threonine kinase activity",
  "gene_symbol": "PRKCE"
}